regulation of actin filament severing [GO:1903918] (biological process) Relationships: is a type of regulation of actin filament-based process [GO:0032970]; regulates GO:0051014 Subtypes: negative regulation of actin filament severing [GO:1903919], GO:1903920 Also known as: regulation of F-actin severing, regulation of actin filament severing activity, regulation of barbed-end actin capping/severing activity Definition: Any process that modulates the frequency, rate or extent of actin filament severing. References: PMID:23325791 Sources: GOC:TermGenie, GOC:als, GO_REF:0000058